{
  "term_id": "UNKNOWN:0003",
  "gene_symbol": "DBI",
  "gene_name": "Acyl-CoA-binding protein",
  "term_label": "Unknown cellular component",
  "gene": "UniProtKB:P07108"
}